{
  "term_id": "GO:2000042",
  "term_label": "negative regulation of double-strand break repair via homologous recombination",
  "gene_symbol": "KLHL15",
  "gene_name": "Kelch-like protein 15",
  "gene": "UniProtKB:Q96M94"
}